regulation of AMPA receptor activity [GO:2000311] (BP) Subtypes: GO:2000969 Sources: GOC:BHF Relationships: is a type of regulation of transmembrane transporter activity [GO:0022898]; is a type of regulation of neurotransmitter receptor activity [GO:0099601]; regulates GO:0004971 Definition: Any process that modulates the frequency, rate or extent of AMPA selective glutamate receptor activity. Also known as: regulation of alpha-amino-3-hydroxy-5-methyl-4-isoxazole propionate selective glutamate receptor activity